peptidyl-arginine methylation, to symmetrical-dimethyl arginine [GO:0019918] (biological process) Sources: RESID:AA0067, RESID:AA0069 Relationships: is_a GO:0035247 Definition: The process of methylation of peptidyl-arginine to form peptidyl-N(omega),N'(omega)-dimethyl-L-arginine.